{
  "gene_name": "Voltage-dependent L-type calcium channel subunit beta-4",
  "term_label": "high voltage-gated calcium channel activity",
  "term_id": "GO:0008331",
  "gene_symbol": "CACNB4",
  "gene": "UniProtKB:O00305"
}